{
  "gene_name": "E3 ubiquitin-protein ligase RNF149",
  "gene": "UniProtKB:Q8NC42",
  "gene_symbol": "RNF149",
  "term_label": "ubiquitin-dependent protein catabolic process",
  "term_id": "GO:0006511"
}